DNA-3'-diphospho-5'-guanosine diphosphatase activity [GO:0120108] (molecular function) Also known as: DNA-3'pp5'G guanylate hydrolase Relationships: is a type of GO:0016462 Definition: Catalysis of the reaction: a 3'-end 2'-deoxyribonucleotide-3'-diphospho-5'-guanosine-DNA + H2O = a 3'-end 2'-deoxyribonucleotide 3'-phosphate-DNA + GMP + 2 H+. References: PMID:26007660 Sources: RHEA:52140